{
  "gene_name": "Beta-defensin 125",
  "gene": "UniProtKB:Q8N687",
  "gene_symbol": "DEFB125",
  "term_label": "innate immune response",
  "term_id": "GO:0045087"
}